oligodendrocyte differentiation [GO:0048709] (biological process) Subtypes: spinal cord oligodendrocyte cell differentiation [GO:0021529], oligodendrocyte cell fate commitment [GO:0021779] Relationships: is_a glial cell differentiation [GO:0010001]; is part of central nervous system development [GO:0007417] References: PMID:15139015 Sources: GOC:vp Regulation: RO_0002211 by regulation of oligodendrocyte differentiation [GO:0048713]; positively regulated by positive regulation of oligodendrocyte differentiation [GO:0048714]; negatively regulated by GO:0048715 Definition: The process in which a relatively unspecialized cell acquires the specialized features of an oligodendrocyte. An oligodendrocyte is a type of glial cell involved in myelinating the axons of neurons in the central nervous system.